{
  "gene": "UniProtKB:Q9BSK0",
  "term_id": "GO:0042552",
  "gene_symbol": "MARVELD1",
  "gene_name": "MARVEL domain-containing protein 1",
  "term_label": "myelination"
}